positive regulation of response to water deprivation [GO:1902584] (biological process) Relationships: is a type of positive regulation of response to stimulus [GO:0048584]; is a type of GO:2000070; positively regulates response to water deprivation [GO:0009414] References: PMID:24198318 Sources: GOC:TermGenie, GO_REF:0000058 Definition: Any process that activates or increases the frequency, rate or extent of response to water deprivation. Also known as: positive regulation of response to dehydration, positive regulation of response to drought, positive regulation of response to thirst, up regulation of response to dehydration, up regulation of response to drought, up regulation of response to thirst, up regulation of response to water deprivation, up-regulation of response to dehydration, up-regulation of response to drought, up-regulation of response to thirst, up-regulation of response to water deprivation, upregulation of response to dehydration, upregulation of response to drought, upregulation of response to thirst, upregulation of response to water deprivation, activation of response to dehydration, activation of response to drought, activation of response to thirst, activation of response to water deprivation, activation of drought tolerance, positive regulation of drought tolerance, up regulation of drought tolerance, up-regulation of drought tolerance, upregulation of drought tolerance